{
  "gene": "UniProtKB:O76094",
  "gene_name": "Signal recognition particle subunit SRP72",
  "term_label": "ribosome binding",
  "gene_symbol": "SRP72",
  "term_id": "GO:0043022"
}